{
  "term_id": "GO:0030141",
  "gene_name": "Transmembrane protease serine 4",
  "gene_symbol": "TMPRSS4",
  "term_label": "secretory granule",
  "gene": "UniProtKB:Q9NRS4"
}